{
  "gene": "UniProtKB:Q7Z713",
  "term_id": "GO:0005737",
  "gene_symbol": "ANKRD37",
  "term_label": "cytoplasm",
  "gene_name": "Ankyrin repeat domain-containing protein 37"
}